{
  "gene_name": "Elongation factor 2",
  "term_id": "GO:0006414",
  "gene": "UniProtKB:P13639",
  "term_label": "translational elongation",
  "gene_symbol": "EEF2"
}